{
  "term_id": "GO:0051018",
  "gene": "UniProtKB:Q02040",
  "gene_symbol": "AKAP17A",
  "gene_name": "A-kinase anchor protein 17A",
  "term_label": "protein kinase A binding"
}